{
  "gene": "UniProtKB:Q8N5X7",
  "gene_name": "Eukaryotic translation initiation factor 4E type 3",
  "term_id": "GO:0016281",
  "term_label": "eukaryotic translation initiation factor 4F complex",
  "gene_symbol": "EIF4E3"
}